positive regulation of mesenchymal stem cell migration [GO:1905322] (biological process) Relationships: is a type of positive regulation of cell migration [GO:0030335]; is a type of regulation of mesenchymal stem cell migration [GO:1905320]; positively regulates mesenchymal stem cell migration [GO:1905319] Also known as: up regulation of mesenchymal stem cell migration, up-regulation of mesenchymal stem cell migration, upregulation of mesenchymal stem cell migration, activation of mesenchymal stem cell migration References: PMID:26846297 Sources: GOC:TermGenie, GO_REF:0000058 Definition: Any process that activates or increases the frequency, rate or extent of mesenchymal stem cell migration.